{
  "term_id": "UNKNOWN:0002",
  "term_label": "Unknown biological process",
  "gene_name": "Protein tweety homolog 3",
  "gene_symbol": "TTYH3",
  "gene": "UniProtKB:Q9C0H2"
}